{
  "term_id": "UNKNOWN:0002",
  "gene_name": "Putative uncharacterized protein FAM120A2P",
  "term_label": "Unknown biological process",
  "gene": "UniProtKB:Q5T035",
  "gene_symbol": "FAM120A2P"
}